{
  "term_id": "GO:0003700",
  "gene": "UniProtKB:O75626",
  "gene_symbol": "PRDM1",
  "gene_name": "PR domain zinc finger protein 1",
  "term_label": "DNA-binding transcription factor activity"
}